{
  "gene": "UniProtKB:Q8IV04",
  "term_label": "retrograde transport, endosome to Golgi",
  "gene_symbol": "TBC1D10C",
  "gene_name": "Carabin",
  "term_id": "GO:0042147"
}